{
  "gene": "UniProtKB:Q5T1A1",
  "gene_symbol": "DCST2",
  "term_label": "Unknown molecular function",
  "gene_name": "DC-STAMP domain-containing protein 2",
  "term_id": "UNKNOWN:0001"
}